{
  "gene_name": "Beta-crystallin B1",
  "term_id": "GO:0007601",
  "gene_symbol": "CRYBB1",
  "term_label": "visual perception",
  "gene": "UniProtKB:P53674"
}